{
  "term_label": "Unknown molecular function",
  "term_id": "UNKNOWN:0001",
  "gene_name": "Ankyrin repeat domain-containing protein 62",
  "gene_symbol": "ANKRD62",
  "gene": "UniProtKB:A6NC57"
}